ATP-dependent peptidase activity [GO:0004176] (molecular function) Relationships: is_a peptidase activity [GO:0008233]; is a type of ATP-dependent activity [GO:0140657] Sources: GOC:mah Definition: Catalysis of the hydrolysis of peptide bonds, driven by ATP hydrolysis. Also known as: ATP-dependent proteolysis